{
  "gene_symbol": "SLC35B4",
  "gene_name": "Nucleotide sugar transporter SLC35B4",
  "gene": "UniProtKB:Q969S0",
  "term_label": "Golgi membrane",
  "term_id": "GO:0000139"
}